{
  "term_id": "UNKNOWN:0001",
  "gene_symbol": "FGB",
  "gene_name": "Fibrinogen beta chain",
  "gene": "UniProtKB:P02675",
  "term_label": "Unknown molecular function"
}